{
  "term_label": "regulation of endocytosis",
  "gene_name": "RUN and FYVE domain-containing protein 1",
  "gene_symbol": "RUFY1",
  "gene": "UniProtKB:Q96T51",
  "term_id": "GO:0030100"
}